{
  "gene_name": "Zinc finger protein 595",
  "term_id": "GO:0006357",
  "gene": "UniProtKB:Q8IYB9",
  "term_label": "regulation of transcription by RNA polymerase II",
  "gene_symbol": "ZNF595"
}